{
  "term_label": "plasma membrane",
  "gene": "UniProtKB:O94823",
  "term_id": "GO:0005886",
  "gene_symbol": "ATP10B",
  "gene_name": "Phospholipid-transporting ATPase VB"
}